{
  "gene_name": "G1_S-specific cyclin-E2",
  "term_id": "GO:1900087",
  "gene_symbol": "CCNE2",
  "gene": "UniProtKB:O96020",
  "term_label": "positive regulation of G1/S transition of mitotic cell cycle"
}